type II interferon receptor binding [GO:0005133] (molecular function) Sources: GOC:ai Definition: Binding to a type II interferon receptor. Type II interferon is also known as interferon-gamma. Relationships: is a type of GO:0005126 Also known as: interferon-gamma receptor binding, interferon-gamma, interferon-gamma receptor ligand